{
  "gene": "UniProtKB:Q96JM3",
  "term_id": "GO:0005819",
  "gene_symbol": "CHAMP1",
  "term_label": "spindle",
  "gene_name": "Chromosome alignment-maintaining phosphoprotein 1"
}